{
  "gene_name": "Gonadotropin-releasing hormone receptor",
  "term_label": "gonadotropin-releasing hormone receptor activity",
  "gene": "UniProtKB:P30968",
  "gene_symbol": "GNRHR",
  "term_id": "GO:0004968"
}